{
  "gene": "UniProtKB:Q7RTY3",
  "term_id": "GO:0004252",
  "term_label": "serine-type endopeptidase activity",
  "gene_symbol": "PRSS45P",
  "gene_name": "Putative serine protease 45"
}